negative regulation of mesodermal cell fate specification [GO:0042662] (biological process) Also known as: down regulation of mesodermal cell fate specification, down-regulation of mesodermal cell fate specification, downregulation of mesodermal cell fate specification, suppression of mesodermal cell fate, inhibition of mesodermal cell fate specification Sources: GOC:go_curators Definition: Any process that stops, prevents, or reduces the frequency, rate or extent of mesoderm cell fate specification. Subtypes: negative regulation of axial mesodermal cell fate specification [GO:0048329], negative regulation of paraxial mesodermal cell fate specification [GO:0048351], negative regulation of lateral mesodermal cell fate specification [GO:0048380], negative regulation of intermediate mesodermal cell fate specification [GO:0048401] Relationships: is a type of GO:0009996; is a type of regulation of mesodermal cell fate specification [GO:0042661]; is a type of negative regulation of mesodermal cell differentiation [GO:1905771]; negatively regulates mesodermal cell fate specification [GO:0007501]